{
  "gene": "UniProtKB:Q8WXT5",
  "gene_name": "Forkhead box protein D4-like 4",
  "term_id": "GO:0000978",
  "term_label": "RNA polymerase II cis-regulatory region sequence-specific DNA binding",
  "gene_symbol": "FOXD4L4"
}